{
  "gene_name": "10 kDa heat shock protein, mitochondrial",
  "gene": "UniProtKB:P61604",
  "gene_symbol": "HSPE1",
  "term_id": "GO:0051087",
  "term_label": "protein-folding chaperone binding"
}